{
  "gene_symbol": "PSG11",
  "gene_name": "Pregnancy-specific beta-1-glycoprotein 11",
  "term_id": "UNKNOWN:0001",
  "term_label": "Unknown molecular function",
  "gene": "UniProtKB:Q9UQ72"
}